{
  "term_id": "GO:0042572",
  "gene_symbol": "ADH6",
  "term_label": "retinol metabolic process",
  "gene": "UniProtKB:P28332",
  "gene_name": "Alcohol dehydrogenase 6"
}